{
  "gene_name": "Aromatic-L-amino-acid decarboxylase",
  "gene_symbol": "DDC",
  "term_id": "GO:0004058",
  "term_label": "aromatic-L-amino-acid decarboxylase activity",
  "gene": "UniProtKB:P20711"
}